antigen processing and presentation, exogenous lipid antigen via MHC class Ib [GO:0048007] (biological process) Also known as: antigen presentation, exogenous peptide antigen, exogenous lipid antigen processing and presentation via MHC class Ib Relationships: is a type of antigen processing and presentation of exogenous antigen [GO:0019884]; is a type of antigen processing and presentation of lipid antigen via MHC class Ib [GO:0048003] References: PMID:10375559, PMID:15928678, PMID:15928680 Sources: GOC:add Definition: The process in which an antigen-presenting cell expresses lipid antigen of exogenous origin in association with an MHC class Ib protein complex on its cell surface. Class Ib here refers to non-classical class I molecules, such as those of the CD1 family.